{
  "gene": "UniProtKB:Q9HAP6",
  "gene_name": "Protein lin-7 homolog B",
  "term_id": "GO:0005911",
  "term_label": "cell-cell junction",
  "gene_symbol": "LIN7B"
}